{
  "term_label": "Unknown biological process",
  "gene_name": "Vesicle transport protein GOT1B",
  "gene": "UniProtKB:Q9Y3E0",
  "gene_symbol": "GOLT1B",
  "term_id": "UNKNOWN:0002"
}